{
  "gene": "UniProtKB:Q96CT2",
  "gene_name": "Kelch-like protein 29",
  "gene_symbol": "KLHL29",
  "term_id": "GO:0031463",
  "term_label": "Cul3-RING ubiquitin ligase complex"
}